pyridoxamine-oxaloacetate transaminase activity [GO:0019162] (molecular function) Sources: EC:2.6.1.31, RHEA:10844 Definition: Catalysis of the reaction: oxaloacetate + pyridoxamine = L-aspartate + pyridoxal. Also known as: pyridoxamine-oxaloacetate aminotransferase activity, pyridoxamine--oxaloacetate aminotransferase activity, pyridoxamine:oxaloacetate aminotransferase activity Relationships: is a type of transaminase activity [GO:0008483]